{
  "term_id": "GO:0006355",
  "term_label": "regulation of DNA-templated transcription",
  "gene": "UniProtKB:Q8TDG2",
  "gene_symbol": "ACTRT1",
  "gene_name": "Actin-related protein T1"
}